{
  "gene": "UniProtKB:P06748",
  "term_id": "GO:1990904",
  "gene_symbol": "NPM1",
  "gene_name": "Nucleophosmin",
  "term_label": "ribonucleoprotein complex"
}